{
  "gene": "UniProtKB:Q5W111",
  "gene_name": "SPRY domain-containing protein 7",
  "term_label": "Unknown cellular component",
  "term_id": "UNKNOWN:0003",
  "gene_symbol": "SPRYD7"
}